{
  "gene_name": "Olfactory receptor 51F1",
  "gene": "UniProtKB:A6NGY5",
  "gene_symbol": "OR51F1",
  "term_id": "UNKNOWN:0002",
  "term_label": "Unknown biological process"
}